root meristem specification [GO:0010071] (biological process) Definition: The specification of a meristem which will give rise to a primary or lateral root. Relationships: is a type of developmental process involved in reproduction [GO:0003006]; is a type of GO:0090421; is part of root morphogenesis [GO:0010015]; is part of GO:0048508 Sources: GOC:ascb_2009, GOC:dph, GOC:tb